{
  "gene_name": "Ankyrin repeat domain-containing protein 31",
  "gene_symbol": "ANKRD31",
  "term_label": "Unknown cellular component",
  "term_id": "UNKNOWN:0003",
  "gene": "UniProtKB:Q8N7Z5"
}